{
  "gene": "UniProtKB:Q9Y238",
  "term_id": "GO:0005737",
  "gene_symbol": "DLEC1",
  "gene_name": "Deleted in lung and esophageal cancer protein 1",
  "term_label": "cytoplasm"
}